cell maturation [GO:0048469] (biological process) Definition: The cellular developmental process, independent of morphogenetic (shape) change, that is required for a specific cell to attain its fully functional state. Also known as: functional differentiation Regulation: regulated by regulation of cell maturation [GO:1903429]; negatively regulated by negative regulation of cell maturation [GO:1903430]; positively regulated by GO:1903431 Relationships: is a type of cellular developmental process [GO:0048869]; is a type of anatomical structure maturation [GO:0071695]; is part of cell development [GO:0048468] Sources: GOC:go_curators Subtypes: oocyte maturation [GO:0001556], epithelial cell maturation [GO:0002070], oocyte construction [GO:0007308], osteoclast maturation [GO:0036179], GO:0036345, neuron maturation [GO:0042551], erythrocyte maturation [GO:0043249], sperm capacitation [GO:0048240], myoblast maturation [GO:0048628], trichoblast maturation [GO:0048764], GO:0090380